first cell cycle pseudocleavage [GO:0030590] (biological process) Definition: A process that occurs during the first cell cycle in an embryo, in which anterior cortical contractions culminate in a single partial constriction of the embryo called the pseudocleavage furrow. An example of this process is found in nematode worms. Relationships: is a type of pseudocleavage [GO:0030588] References: PMID:7729583 Sources: GOC:mtg_sensu